protein localization to actin cortical patch [GO:0044379] (biological process) Definition: A process in which a protein is transported to, or maintained in, an actin cortical patch. Regulation: regulated by regulation of protein localization to actin cortical patch [GO:1904370]; negatively regulated by negative regulation of protein localization to actin cortical patch [GO:1904371]; positively regulated by positive regulation of protein localization to actin cortical patch [GO:1904372] Also known as: protein localisation to actin cortical patch Relationships: is a type of protein localization to cell cortex [GO:0072697]; is a type of protein localization to actin cytoskeleton [GO:1903119] References: PMID:21620704 Sources: GOC:mah